{
  "gene_symbol": "ZBTB20",
  "gene": "UniProtKB:Q9HC78",
  "gene_name": "Zinc finger and BTB domain-containing protein 20",
  "term_id": "GO:0005654",
  "term_label": "nucleoplasm"
}